{
  "term_id": "GO:0016208",
  "gene_symbol": "PRKAG1",
  "gene_name": "5'-AMP-activated protein kinase subunit gamma-1",
  "gene": "UniProtKB:P54619",
  "term_label": "AMP binding"
}